{
  "term_label": "lens development in camera-type eye",
  "gene_symbol": "CRYBG3",
  "term_id": "GO:0002088",
  "gene": "UniProtKB:Q68DQ2",
  "gene_name": "Very large A-kinase anchor protein"
}